{
  "term_id": "GO:0044545",
  "gene_name": "Histone acetyltransferase KAT8",
  "gene": "UniProtKB:Q9H7Z6",
  "gene_symbol": "KAT8",
  "term_label": "NSL complex"
}